tRNA (guanine(7)-N2)-methyltransferase activity [GO:0160118] (molecular function) Relationships: is a type of N-methyltransferase activity [GO:0008170]; is a type of GO:0016423 Definition: Catalysis of the reaction: guanosine(7) in tRNA + S-adenosyl-L-methionine = H+ + N(2)-methylguanosine(7) in tRNA + S-adenosyl-L-homocysteine. References: PMID:34669960